{
  "gene_symbol": "TAOK2",
  "term_id": "GO:0032874",
  "term_label": "positive regulation of stress-activated MAPK cascade",
  "gene": "UniProtKB:Q9UL54",
  "gene_name": "Serine_threonine-protein kinase TAO2"
}